{
  "gene": "UniProtKB:P42229",
  "gene_symbol": "STAT5A",
  "gene_name": "Signal transducer and activator of transcription 5A",
  "term_label": "cytokine-mediated signaling pathway",
  "term_id": "GO:0019221"
}